{
  "term_label": "regulation of transcription by RNA polymerase II",
  "term_id": "GO:0006357",
  "gene_name": "Factor in the germline alpha",
  "gene_symbol": "FIGLA",
  "gene": "UniProtKB:Q6QHK4"
}